{
  "gene_symbol": "GABRA3",
  "gene": "UniProtKB:P34903",
  "gene_name": "Gamma-aminobutyric acid receptor subunit alpha-3",
  "term_id": "GO:1904862",
  "term_label": "inhibitory synapse assembly"
}